{
  "gene": "UniProtKB:P0CB38",
  "gene_name": "Polyadenylate-binding protein 4-like",
  "gene_symbol": "PABPC4L",
  "term_id": "UNKNOWN:0002",
  "term_label": "Unknown biological process"
}